{
  "term_label": "Unknown cellular component",
  "gene_symbol": "CATIP",
  "term_id": "UNKNOWN:0003",
  "gene": "UniProtKB:Q7Z7H3",
  "gene_name": "Ciliogenesis-associated TTC17-interacting protein"
}